{
  "gene_name": "Unconventional myosin-Id",
  "gene": "UniProtKB:O94832",
  "term_label": "microfilament motor activity",
  "term_id": "GO:0000146",
  "gene_symbol": "MYO1D"
}